adenosylcobyric acid synthase (glutamine-hydrolyzing) activity [GO:0051921] (molecular function) Also known as: CobQ activity, 5'-deoxy-5'-adenosylcobyrinic-acid-a,c-diamide:L-glutamine amido-ligase activity, Ado-cobyric acid synthase [glutamine hydrolyzing] activity, adenosylcobyric acid synthase (glutamine-hydrolysing) activity, adenosylcobyrinic-acid-a,c-diamide:L-glutamine amido-ligase (ADP-forming), cobyric acid synthase activity Relationships: is a type of GO:0016884 Sources: EC:6.3.5.10, RHEA:23256 Definition: Catalysis of the reaction: 4 L-glutamine + adenosylcob(III)yrinate a,c-diamide + 4 ATP + 4 H2O = 4 L-glutamate + adenosylcobyrate + 4 ADP + 8 H+ + 4 phosphate.